positive regulation of supramolecular fiber organization [GO:1902905] (biological process) References: PMID:23921388 Sources: GOC:PARL, GOC:TermGenie, GOC:rl, GO_REF:0000058 Subtypes: positive regulation of actin filament depolymerization [GO:0030836], positive regulation of actin filament polymerization [GO:0030838], positive regulation of microtubule polymerization [GO:0031116], GO:0031117, positive regulation of actin filament bundle assembly [GO:0032233], GO:0051127, GO:0060298, positive regulation of myosin II filament organization [GO:1904901], positive regulation of cardiac myofibril assembly [GO:1905306], positive regulation of amyloid fibril formation [GO:1905908] Definition: Any process that activates or increases the frequency, rate or extent of supramolecular fiber organization. Note: HSPA8, human, P11142 in PMID:23921388 inferred from direct assay to negatively regulate fibrillation of alpha-Syn in vitro Relationships: is a type of GO:0051130; is a type of regulation of supramolecular fiber organization [GO:1902903]; positively regulates supramolecular fiber organization [GO:0097435] Also known as: activation of fibril organisation, activation of fibril organization, positive regulation of fibril organisation, up regulation of fibril organisation, up regulation of fibril organization, up-regulation of fibril organisation, up-regulation of fibril organization, upregulation of fibril organisation, upregulation of fibril organization